{
  "term_id": "GO:0005829",
  "gene_symbol": "HSPA2",
  "gene": "UniProtKB:P54652",
  "term_label": "cytosol",
  "gene_name": "Heat shock-related 70 kDa protein 2"
}